{
  "term_id": "GO:0045943",
  "gene_name": "Nucleolar transcription factor 1",
  "gene_symbol": "UBTF",
  "term_label": "positive regulation of transcription by RNA polymerase I",
  "gene": "UniProtKB:P17480"
}